{
  "gene": "UniProtKB:E2RYF7",
  "term_id": "UNKNOWN:0003",
  "gene_symbol": "HCG22",
  "term_label": "Unknown cellular component",
  "gene_name": "Protein PBMUCL2"
}